{
  "gene_symbol": "C1QTNF4",
  "term_id": "UNKNOWN:0001",
  "term_label": "Unknown molecular function",
  "gene_name": "Complement C1q tumor necrosis factor-related protein 4",
  "gene": "UniProtKB:Q9BXJ3"
}